lateral sprouting involved in lung morphogenesis [GO:0060490] (biological process) Definition: The process in which a branch forms along the side of the lung epithelial tube. Relationships: is a type of lateral sprouting from an epithelium [GO:0060601]; is part of epithelial tube branching involved in lung morphogenesis [GO:0060441] Sources: GOC:dph, GOC:mtg_lung